{
  "term_label": "RNA polymerase II cis-regulatory region sequence-specific DNA binding",
  "gene_symbol": "ZBTB9",
  "gene_name": "Zinc finger and BTB domain-containing protein 9",
  "term_id": "GO:0000978",
  "gene": "UniProtKB:Q96C00"
}